{
  "gene_symbol": "C1QTNF4",
  "gene": "UniProtKB:Q9BXJ3",
  "term_id": "GO:1901224",
  "gene_name": "Complement C1q tumor necrosis factor-related protein 4",
  "term_label": "positive regulation of non-canonical NF-kappaB signal transduction"
}